{
  "term_label": "Unknown biological process",
  "gene_name": "Apoptosis-stimulating of p53 protein 1",
  "gene_symbol": "PPP1R13B",
  "gene": "UniProtKB:Q96KQ4",
  "term_id": "UNKNOWN:0002"
}